Golgi calcium ion transport [GO:0032472] (BP) Definition: The directed movement of calcium ions (Ca2+) into, out of or within the Golgi apparatus. Subtypes: GO:0061856 Also known as: Golgi calcium transport Relationships: is a type of GO:0006816 Sources: GOC:mah